nuclear envelope organization [GO:0006998] (biological process) Relationships: is a type of membrane organization [GO:0061024]; is part of GO:0006997; is part of endomembrane system organization [GO:0010256] Also known as: nuclear envelope organisation, nuclear envelope organization and biogenesis Sources: GOC:dph, GOC:ems, GOC:jl, GOC:mah Subtypes: pronuclear envelope synthesis [GO:0018985] Definition: A process that is carried out at the cellular level which results in the assembly, arrangement of constituent parts, or disassembly of the nuclear envelope.